{
  "gene_name": "Transmembrane protein 131",
  "term_id": "UNKNOWN:0002",
  "term_label": "Unknown biological process",
  "gene": "UniProtKB:Q92545",
  "gene_symbol": "TMEM131"
}